{
  "gene_name": "von Willebrand factor A domain-containing protein 8",
  "term_id": "UNKNOWN:0001",
  "gene": "UniProtKB:A3KMH1",
  "gene_symbol": "VWA8",
  "term_label": "Unknown molecular function"
}